{
  "gene": "UniProtKB:Q6ZVL6",
  "gene_symbol": "KIAA1549L",
  "gene_name": "UPF0606 protein KIAA1549L",
  "term_id": "UNKNOWN:0001",
  "term_label": "Unknown molecular function"
}